{
  "term_label": "Unknown cellular component",
  "gene_symbol": "C6orf120",
  "term_id": "UNKNOWN:0003",
  "gene_name": "UPF0669 protein C6orf120",
  "gene": "UniProtKB:Q7Z4R8"
}